{
  "term_label": "protein localization to endoplasmic reticulum exit site",
  "gene_name": "B-cell receptor-associated protein 31",
  "gene": "UniProtKB:P51572",
  "gene_symbol": "BCAP31",
  "term_id": "GO:0070973"
}